{
  "gene_symbol": "MYO19",
  "term_id": "GO:0007015",
  "gene": "UniProtKB:Q96H55",
  "gene_name": "Unconventional myosin-XIX",
  "term_label": "actin filament organization"
}